{
  "term_id": "GO:0043001",
  "gene_symbol": "GOLPH3L",
  "gene_name": "Golgi phosphoprotein 3-like",
  "term_label": "Golgi to plasma membrane protein transport",
  "gene": "UniProtKB:Q9H4A5"
}